regulation of hair follicle development [GO:0051797] (biological process) Sources: GOC:ai Definition: Any process that modulates the frequency, rate or extent of hair follicle development. Relationships: is a type of GO:0042634; is a type of regulation of multicellular organismal development [GO:2000026]; regulates GO:0001942 Subtypes: GO:0051798, negative regulation of hair follicle development [GO:0051799]